{
  "gene_name": "Pleckstrin homology domain-containing family A member 7",
  "gene": "UniProtKB:Q6IQ23",
  "term_id": "UNKNOWN:0001",
  "term_label": "Unknown molecular function",
  "gene_symbol": "PLEKHA7"
}